{
  "gene_symbol": "IL23A",
  "term_id": "GO:0002230",
  "term_label": "positive regulation of defense response to virus by host",
  "gene": "UniProtKB:Q9NPF7",
  "gene_name": "Interleukin-23 subunit alpha"
}